{
  "gene_symbol": "TPST2",
  "gene_name": "Protein-tyrosine sulfotransferase 2",
  "gene": "UniProtKB:O60704",
  "term_label": "protein-tyrosine sulfotransferase activity",
  "term_id": "GO:0008476"
}